{
  "term_id": "UNKNOWN:0001",
  "gene_name": "Peptidase inhibitor R3HDML",
  "gene_symbol": "R3HDML",
  "gene": "UniProtKB:Q9H3Y0",
  "term_label": "Unknown molecular function"
}